positive regulation of glomerular filtration [GO:0003104] (biological process) Relationships: is a type of regulation of glomerular filtration [GO:0003093]; is a type of positive regulation of multicellular organismal process [GO:0051240]; positively regulates glomerular filtration [GO:0003094] Sources: GOC:mtg_cardio Definition: Any process that activates or increases the frequency, rate or extent of glomerular filtration. Glomerular filtration is the process whereby blood is filtered by the glomerulus into the renal tubule.